positive regulation of amide metabolic process [GO:0034250] (biological process) Subtypes: positive regulation of penicillin metabolic process [GO:0033246], GO:0034253, GO:0060569, positive regulation of pyruvate decarboxylation to acetyl-CoA [GO:0140176], positive regulation of isopentenyl diphosphate biosynthetic process, mevalonate pathway [GO:1900486], GO:1900496, positive regulation of butyryl-CoA catabolic process to butanol [GO:1900499], positive regulation of butyryl-CoA catabolic process to butyrate [GO:1900502], positive regulation of emericellamide biosynthetic process [GO:1900660], positive regulation of gliotoxin biosynthetic process [GO:1900691], positive regulation of tensidol A biosynthetic process [GO:1900709], GO:1900712, positive regulation of pseurotin A biosynthetic process [GO:1900851], GO:1901415, GO:1902004, GO:1903788, positive regulation of ferrichrome biosynthetic process [GO:1905570], GO:2000304, positive regulation of glucosylceramide catabolic process [GO:2000753], positive regulation of sphingomyelin catabolic process [GO:2000755] Definition: Any process that activates or increases the frequency, rate or extent of the chemical reactions and pathways involving amides. Also known as: positive regulation of amide metabolism, positive regulation of cellular amide metabolic process Sources: GOC:mah Relationships: is a type of positive regulation of metabolic process [GO:0009893]; is a type of GO:0034248; positively regulates amide metabolic process [GO:0043603]